{
  "term_id": "GO:0005737",
  "gene": "UniProtKB:Q96GR2",
  "gene_name": "Long-chain-fatty-acid--CoA ligase ACSBG1",
  "gene_symbol": "ACSBG1",
  "term_label": "cytoplasm"
}